{
  "term_label": "Unknown biological process",
  "term_id": "UNKNOWN:0002",
  "gene_name": "Tigger transposable element-derived protein 1",
  "gene": "UniProtKB:Q96MW7",
  "gene_symbol": "TIGD1"
}